{
  "term_label": "regulation of actin cytoskeleton organization",
  "gene_symbol": "ARHGEF26",
  "gene_name": "Rho guanine nucleotide exchange factor 26",
  "gene": "UniProtKB:Q96DR7",
  "term_id": "GO:0032956"
}